{
  "term_label": "animal organ development",
  "gene_name": "Somatotropin",
  "gene": "UniProtKB:P01241",
  "term_id": "GO:0048513",
  "gene_symbol": "GH1"
}